{
  "term_id": "GO:0071763",
  "gene_name": "LEM domain-containing protein 2",
  "gene_symbol": "LEMD2",
  "term_label": "nuclear membrane organization",
  "gene": "UniProtKB:Q8NC56"
}